{
  "term_id": "GO:0031011",
  "gene_symbol": "RUVBL2",
  "gene_name": "RuvB-like 2",
  "gene": "UniProtKB:Q9Y230",
  "term_label": "Ino80 complex"
}